{
  "gene_symbol": "TXNDC2",
  "gene": "UniProtKB:Q86VQ3",
  "gene_name": "Thioredoxin domain-containing protein 2",
  "term_id": "UNKNOWN:0002",
  "term_label": "Unknown biological process"
}